{
  "gene": "UniProtKB:Q6ZSZ6",
  "gene_name": "Teashirt homolog 1",
  "term_id": "GO:0006357",
  "gene_symbol": "TSHZ1",
  "term_label": "regulation of transcription by RNA polymerase II"
}